{
  "gene_name": "Arfaptin-1",
  "term_id": "GO:0005543",
  "term_label": "phospholipid binding",
  "gene_symbol": "ARFIP1",
  "gene": "UniProtKB:P53367"
}